{
  "gene_symbol": "RRBP1",
  "gene_name": "Ribosome-binding protein 1",
  "term_label": "endoplasmic reticulum membrane",
  "term_id": "GO:0005789",
  "gene": "UniProtKB:Q9P2E9"
}